{
  "term_id": "GO:0005912",
  "gene": "UniProtKB:Q9NYQ7",
  "term_label": "adherens junction",
  "gene_symbol": "CELSR3",
  "gene_name": "Cadherin EGF LAG seven-pass G-type receptor 3"
}